{
  "term_label": "mitochondrial outer membrane translocase complex assembly",
  "gene_name": "Metaxin-2",
  "gene": "UniProtKB:O75431",
  "gene_symbol": "MTX2",
  "term_id": "GO:0070096"
}